{
  "gene_name": "Kelch-like protein 40",
  "term_id": "GO:0031397",
  "gene": "UniProtKB:Q2TBA0",
  "term_label": "negative regulation of protein ubiquitination",
  "gene_symbol": "KLHL40"
}